{
  "gene_name": "Potassium voltage-gated channel subfamily D member 3",
  "gene_symbol": "KCND3",
  "gene": "UniProtKB:Q9UK17",
  "term_label": "dendritic spine",
  "term_id": "GO:0043197"
}